{
  "gene": "UniProtKB:A0A0A0MT82",
  "gene_name": "Immunoglobulin lambda joining 2 (Fragment)",
  "gene_symbol": "IGLJ2",
  "term_id": "UNKNOWN:0001",
  "term_label": "Unknown molecular function"
}